EGF repeat binding [GO:0061788] (MF) Definition: Binding to Epidermal Growth Factor (EGF) repeats. References: PMID:25155514 Sources: GOC:25700513, GOC:dph Also known as: Epidermal growth factor domain binding, Epidermal Growth Factor repeat binding Relationships: is a type of protein domain specific binding [GO:0019904]